{
  "gene_symbol": "LAMA3",
  "term_id": "GO:0045202",
  "gene": "UniProtKB:Q16787",
  "gene_name": "Laminin subunit alpha-3",
  "term_label": "synapse"
}